polyubiquitinated misfolded protein transport [GO:0070845] (biological process) Definition: The directed movement of misfolded polyubiquitinated proteins in a cell, including the movement of proteins between specific compartments or structures within a cell. References: PMID:14675537 Sources: GOC:BHF, GOC:mah Also known as: polyubiquitylated misfolded protein transport, misfolded polyubiquitinated protein transport Relationships: is a type of GO:0070843; is a type of polyubiquitinated protein transport [GO:0070844]